{
  "gene_name": "PHD finger protein 10",
  "gene": "UniProtKB:Q8WUB8",
  "gene_symbol": "PHF10",
  "term_label": "regulation of transcription by RNA polymerase II",
  "term_id": "GO:0006357"
}